{
  "gene_name": "EF-hand calcium-binding domain-containing protein 9",
  "gene_symbol": "EFCAB9",
  "gene": "UniProtKB:A8MZ26",
  "term_id": "GO:0061891",
  "term_label": "calcium ion sensor activity"
}